alpha-neoagaro-oligosaccharide hydrolase activity [GO:0033954] (molecular function) Relationships: is a type of hydrolase activity, hydrolyzing O-glycosyl compounds [GO:0004553] Sources: EC:3.2.1.159 Also known as: alpha-NAOS hydrolase activity, alpha-neoagaro-oligosaccharide 3-glycohydrolase activity, alpha-neoagarooligosaccharide hydrolase activity Definition: Catalysis of the hydrolysis of the 1,3-alpha-L-galactosidic linkages of neoagaro-oligosaccharides that are smaller than a hexamer, yielding 3,6-anhydro-L-galactose and D-galactose.